regulation of phosphatidylcholine metabolic process [GO:0150172] (biological process) References: PMID:30074985 Sources: GOC:aruk, GOC:bc Definition: Any process that modulates the frequency, rate or extent of phosphatidylcholine metabolic process. Subtypes: GO:0010899, regulation of phosphatidylcholine biosynthetic process [GO:2001245] Relationships: is a type of regulation of phospholipid metabolic process [GO:1903725]; RO_0002211 GO:0046470